alkene catabolic process [GO:0043451] (BP) Relationships: is a type of hydrocarbon catabolic process [GO:0120253]; is a type of GO:0120256; is a type of olefin metabolic process [GO:1900673] Subtypes: propylene catabolic process [GO:0042208], GO:0042457 Definition: The chemical reactions and pathways resulting in the breakdown of an alkene, any acyclic branched or unbranched hydrocarbon having one carbon-carbon double bond and the general formula CnH2n. Sources: GOC:jl, Wikipedia:Alkene Also known as: alkene breakdown, alkene catabolism, alkene degradation